{
  "term_label": "detection of mechanical stimulus",
  "gene": "UniProtKB:Q13563",
  "gene_name": "Polycystin-2",
  "term_id": "GO:0050982",
  "gene_symbol": "PKD2"
}